oocyte fate determination [GO:0030716] (biological process) Relationships: is_a cell fate determination [GO:0001709] Sources: GOC:go_curators Also known as: oocyte cell fate determination Definition: The process in which a cell becomes capable of differentiating autonomously into an oocyte cell regardless of its environment; upon determination, the cell fate cannot be reversed. Subtypes: germarium-derived oocyte fate determination [GO:0007294]